{
  "gene_symbol": "CABYR",
  "term_id": "GO:0005737",
  "gene": "UniProtKB:O75952",
  "gene_name": "Calcium-binding tyrosine phosphorylation-regulated protein",
  "term_label": "cytoplasm"
}